{
  "term_label": "nucleolus",
  "gene_name": "Protein SPT2 homolog",
  "term_id": "GO:0005730",
  "gene_symbol": "SPTY2D1",
  "gene": "UniProtKB:Q68D10"
}